{
  "gene": "UniProtKB:A6ND91",
  "term_id": "UNKNOWN:0002",
  "term_label": "Unknown biological process",
  "gene_name": "Aspartate dehydrogenase domain-containing protein",
  "gene_symbol": "ASPDH"
}